{
  "term_label": "SUMO ligase activity",
  "term_id": "GO:0061665",
  "gene": "UniProtKB:Q8NF64",
  "gene_symbol": "ZMIZ2",
  "gene_name": "Zinc finger MIZ domain-containing protein 2"
}